{
  "gene_name": "Putative uncharacterized protein ENSP00000334305",
  "term_id": "GO:0005886",
  "term_label": "plasma membrane",
  "gene": "UniProtKB:Q3C1V9",
  "gene_symbol": "Q3C1V9"
}